{
  "gene_name": "Uncharacterized protein",
  "term_id": "UNKNOWN:0002",
  "gene": "UniProtKB:A0A6Q8PGL7",
  "term_label": "Unknown biological process",
  "gene_symbol": "A0A6Q8PGL7"
}